{
  "gene": "UniProtKB:Q10567",
  "gene_name": "AP-1 complex subunit beta-1",
  "term_label": "Unknown molecular function",
  "term_id": "UNKNOWN:0001",
  "gene_symbol": "AP1B1"
}